detection of temperature stimulus involved in sensory perception of pain [GO:0050965] (biological process) Definition: The series of events involved in the perception of pain in which a temperature stimulus is received and converted into a molecular signal. Also known as: perception of pain, detection of temperature stimulus, perception of pain, sensory detection of temperature stimulus, perception of pain, sensory transduction of temperature stimulus, sensory detection of temperature stimulus during perception of pain, sensory detection of thermal stimulus during sensory perception of pain, sensory perception of pain, sensory detection of thermal stimulus, sensory perception of pain, sensory transduction of thermal stimulus, sensory transduction of temperature stimulus during perception of pain, sensory transduction of thermal stimulus during sensory perception of pain, thermal nociception Sources: GOC:ai, GOC:dos Relationships: is a type of detection of temperature stimulus involved in sensory perception [GO:0050961]; is a type of detection of stimulus involved in sensory perception of pain [GO:0062149]